(S)-reticuline biosynthetic process [GO:1901012] (biological process) Also known as: (S)-reticuline anabolism, (S)-reticuline biosynthesis, (S)-reticuline formation, (S)-reticuline synthesis References: PMID:22725256 Sources: GOC:TermGenie, GOC:yaf Definition: The chemical reactions and pathways resulting in the formation of (S)-reticuline. Relationships: is a type of benzyl isoquinoline alkaloid biosynthetic process [GO:0009708]